{
  "term_label": "nucleoplasm",
  "gene": "UniProtKB:Q6ZMV5",
  "term_id": "GO:0005654",
  "gene_symbol": "PPP4R3C",
  "gene_name": "Protein PPP4R3C"
}